{
  "term_id": "GO:0030154",
  "gene_symbol": "GSK3B",
  "gene_name": "Glycogen synthase kinase-3 beta",
  "term_label": "cell differentiation",
  "gene": "UniProtKB:P49841"
}